{
  "gene_symbol": "KYAT3",
  "term_id": "GO:0016212",
  "gene_name": "Kynurenine--oxoglutarate transaminase 3",
  "gene": "UniProtKB:Q6YP21",
  "term_label": "kynurenine-oxoglutarate transaminase activity"
}